{
  "gene_name": "Centrosomal protein of 83 kDa",
  "gene": "UniProtKB:Q9Y592",
  "term_id": "GO:0005813",
  "gene_symbol": "CEP83",
  "term_label": "centrosome"
}